{
  "gene": "UniProtKB:Q6PCB5",
  "term_id": "UNKNOWN:0001",
  "gene_name": "Lysine-specific demethylase RSBN1L",
  "term_label": "Unknown molecular function",
  "gene_symbol": "RSBN1L"
}